detection of symbiont [GO:0009602] (biological process) Sources: GOC:hb, ISBN:0198506732 Subtypes: detection of parasitic plant [GO:0002243], detection of symbiotic fungus [GO:0009603], detection of symbiotic bacterium [GO:0009604] Relationships: is a type of response to symbiont [GO:0009608]; is a type of biological process involved in interaction with symbiont [GO:0051702]; is a type of detection of other organism [GO:0098543] Also known as: recognition of symbiont, perception of symbiont Definition: The series of events in which a stimulus from a symbiont (an organism living in close physical association with an organism of a different species) is received and converted into a molecular signal. The symbiont is defined as the smaller of the organisms involved in a symbiotic interaction.